{
  "gene_symbol": "ATP6V1G3",
  "term_label": "vacuolar proton-transporting V-type ATPase, V1 domain",
  "gene_name": "V-type proton ATPase subunit G 3",
  "term_id": "GO:0000221",
  "gene": "UniProtKB:Q96LB4"
}